{
  "gene": "UniProtKB:Q9NS28",
  "gene_symbol": "RGS18",
  "term_id": "GO:0005096",
  "gene_name": "Regulator of G-protein signaling 18",
  "term_label": "GTPase activator activity"
}